trochlear nerve morphogenesis [GO:0021639] (biological process) Relationships: is a type of cranial nerve morphogenesis [GO:0021602]; is part of trochlear nerve development [GO:0021558] Sources: GOC:cls, GOC:dgh, GOC:dph, GOC:jid, GO_REF:0000021 Definition: The process in which the anatomical structure of the trochlear nerve is generated and organized. The trochlear nerve is a motor nerve and is the only cranial nerve to exit the brain dorsally. The trochlear nerve innervates the superior oblique muscle. Also known as: CH IV morphogenesis